{
  "gene": "UniProtKB:Q9NVP2",
  "gene_symbol": "ASF1B",
  "term_id": "GO:0042393",
  "term_label": "histone binding",
  "gene_name": "Histone chaperone ASF1B"
}